{
  "term_label": "chemical synaptic transmission",
  "gene_symbol": "SNCB",
  "gene_name": "Beta-synuclein",
  "gene": "UniProtKB:Q16143",
  "term_id": "GO:0007268"
}